lamin depolymerization [GO:0007078] (biological process) Definition: The cell cycle process in which lamin is depolymerized. Sources: GOC:jid Relationships: is_a protein depolymerization [GO:0051261]; is a type of GO:1903047; is part of mitotic nuclear membrane disassembly [GO:0007077]